ribonuclease E activity [GO:0008995] (molecular function) Also known as: ribonuclease G activity Definition: Catalysis of the cleavage of single-stranded RNA that is monophosphorylated at its 5'-end; cleavage occurs predominantly at 5 nucleotides from the 5'-end and in A + U-rich regions, and is blocked by the presence of a 5'-triphosphate group. Relationships: is a type of RNA endonuclease activity producing 5'-phosphomonoesters, hydrolytic mechanism [GO:0016891] References: PMID:10722715, PMID:16854990 Sources: EC:3.1.26.12